transforming growth factor beta binding [GO:0050431] (molecular function) Sources: ISBN:0198506732 Definition: Binding to TGF-beta, transforming growth factor beta, a multifunctional peptide that controls proliferation, differentiation and other functions in many cell types. Also known as: TGF-beta binding, TGFbeta binding, transforming growth factor beta ligand binding to type I receptor, transforming growth factor beta ligand binding to type II receptor Relationships: is a type of GO:0019838; is a type of cytokine binding [GO:0019955]